{
  "gene": "UniProtKB:Q14318",
  "term_id": "GO:0016020",
  "term_label": "membrane",
  "gene_symbol": "FKBP8",
  "gene_name": "Peptidyl-prolyl cis-trans isomerase FKBP8"
}